amylin receptor signaling pathway [GO:0097647] (biological process) Also known as: amilyn receptor signalling pathway References: PMID:10871296, PMID:12037140, PMID:18687416 Sources: GOC:bhm Relationships: is a type of GO:0097646 Definition: A G protein-coupled receptor signaling pathway initiated by amylin binding to its receptor on the surface of a target cell, and ending with the regulation of a downstream cellular process. Subtypes: amylin receptor 1 signaling pathway [GO:0150059], GO:0150060, amylin receptor 3 signaling pathway [GO:0150061]